microtubule-based movement [GO:0007018] (BP) Relationships: is a type of microtubule-based process [GO:0007017] Regulation: regulated by regulation of microtubule-based movement [GO:0060632] Sources: GOC:cjm, ISBN:0815316194 Subtypes: cilium movement [GO:0003341], GO:0010970, establishment of mitochondrion localization, microtubule-mediated [GO:0034643], microtubule sliding [GO:0051012], chromosome movement towards spindle pole [GO:0051305], microtubule polymerization based movement [GO:0099098], microtubule plus-end directed mitotic chromosome migration [GO:0099606], GO:0140405 Definition: A microtubule-based process that results in the movement of organelles, other microtubules, or other cellular components. Examples include motor-driven movement along microtubules and movement driven by polymerization or depolymerization of microtubules.